{
  "term_id": "GO:0006874",
  "gene_symbol": "STIM1",
  "gene": "UniProtKB:Q13586",
  "term_label": "intracellular calcium ion homeostasis",
  "gene_name": "Stromal interaction molecule 1"
}